tRNA wobble cytosine modification [GO:0002101] (biological process) Relationships: is a type of tRNA wobble base modification [GO:0002097] Definition: The process in which a cytosine at position 34 of a tRNA is post-transcriptionally modified. The wobble nucleoside of the tRNA sequence  (position 34) corresponds to the first position of the anticodon. Subtypes: GO:0002127, tRNA wobble base lysidine biosynthesis [GO:0002136] Sources: GOC:hjd, ISBN:155581073X